{
  "gene_symbol": "PNLIPRP3",
  "gene_name": "Pancreatic lipase-related protein 3",
  "term_label": "high-density lipoprotein particle remodeling",
  "term_id": "GO:0034375",
  "gene": "UniProtKB:Q17RR3"
}